{
  "term_id": "UNKNOWN:0003",
  "gene_name": "Filamin-B",
  "term_label": "Unknown cellular component",
  "gene": "UniProtKB:O75369",
  "gene_symbol": "FLNB"
}